{
  "gene": "UniProtKB:Q6ZVS7",
  "term_label": "Unknown molecular function",
  "gene_symbol": "CFAP144P1",
  "term_id": "UNKNOWN:0001",
  "gene_name": "Protein FAM183BP"
}